{
  "gene": "UniProtKB:Q8N122",
  "gene_name": "Regulatory-associated protein of mTOR",
  "gene_symbol": "RPTOR",
  "term_id": "GO:0030674",
  "term_label": "protein-macromolecule adaptor activity"
}